neuroblast division in subpallium [GO:0021848] (biological process) Also known as: neuroblast division in the ventral telencephalon Definition: The division of neuroblasts in the subpallium area of the forebrain. The interneuron precursors that these cells give rise to include GABAergic interneurons and will migrate tangentially. References: PMID:12626695 Sources: GOC:cls, GOC:dgh, GOC:dph, GOC:jid, GO_REF:0000021 Subtypes: neuroblast division in dorsal lateral ganglionic eminence [GO:0021851] Relationships: is a type of neuroblast division [GO:0055057]; is part of subpallium cell proliferation in forebrain [GO:0022012]